{
  "gene_name": "RING finger and SPRY domain-containing protein 1",
  "term_label": "proteolysis involved in protein catabolic process",
  "term_id": "GO:0051603",
  "gene": "UniProtKB:Q96DX4",
  "gene_symbol": "RSPRY1"
}